{
  "term_label": "regulation of gene expression",
  "gene": "UniProtKB:Q9H9E1",
  "gene_name": "Ankyrin repeat family A protein 2",
  "term_id": "GO:0010468",
  "gene_symbol": "ANKRA2"
}